negative regulation of androgen secretion [GO:2000835] (biological process) Relationships: is_a GO:2000832; is a type of regulation of androgen secretion [GO:2000834]; negatively regulates androgen secretion [GO:0035935] Sources: GOC:sl Definition: Any process that stops, prevents or reduces the frequency, rate or extent of androgen secretion.